{
  "gene_symbol": "BRINP3",
  "gene": "UniProtKB:Q76B58",
  "term_label": "neuronal cell body",
  "gene_name": "BMP_retinoic acid-inducible neural-specific protein 3",
  "term_id": "GO:0043025"
}